{
  "gene_name": "Protein WFDC10B",
  "term_id": "GO:0019731",
  "term_label": "antibacterial humoral response",
  "gene_symbol": "WFDC10B",
  "gene": "UniProtKB:Q8IUB3"
}